inositol-1,2,4,5,6-pentakisphosphate 5-phosphatase activity [GO:1990651] (molecular function) Definition: Catalysis of the reaction: 1D-myo-inositol 1,2,4,5,6-pentakisphosphate + H2O = 1D-myo-inositol 1,2,4,6-tetrakisphosphate + phosphate. References: PMID:15316017 Sources: GOC:al Relationships: is a type of GO:0052827